{
  "gene_name": "Prolyl hydroxylase EGLN3",
  "term_label": "nucleus",
  "gene": "UniProtKB:Q9H6Z9",
  "term_id": "GO:0005634",
  "gene_symbol": "EGLN3"
}